{
  "gene_symbol": "FRMD4A",
  "term_label": "Unknown molecular function",
  "gene": "UniProtKB:Q9P2Q2",
  "gene_name": "FERM domain-containing protein 4A",
  "term_id": "UNKNOWN:0001"
}